{
  "gene": "UniProtKB:Q8N8J0",
  "term_label": "Unknown cellular component",
  "term_id": "UNKNOWN:0003",
  "gene_name": "Putative inactive phosphatidylinositol 4-kinase alpha-like protein P1",
  "gene_symbol": "PI4KAP1"
}